{
  "term_id": "GO:0004674",
  "gene_symbol": "DYRK4",
  "term_label": "protein serine/threonine kinase activity",
  "gene_name": "Dual specificity tyrosine-phosphorylation-regulated kinase 4",
  "gene": "UniProtKB:Q9NR20"
}